{
  "gene_name": "Interferon-induced GTP-binding protein Mx2",
  "term_label": "microtubule binding",
  "term_id": "GO:0008017",
  "gene": "UniProtKB:P20592",
  "gene_symbol": "MX2"
}